valine-tRNA ligase activity [GO:0004832] (molecular function) Definition: Catalysis of the reaction: L-valine + ATP + tRNA(Val) = L-valyl-tRNA(Val) + AMP + diphosphate + 2 H+. Also known as: valyl-tRNA synthetase activity, L-valine:tRNAVal ligase (AMP-forming), valine transfer ribonucleate ligase activity, valine translase activity, valyl-transfer RNA synthetase activity, valyl-transfer ribonucleate synthetase activity, valyl-transfer ribonucleic acid synthetase activity Sources: EC:6.1.1.9, RHEA:10704 Relationships: is a type of aminoacyl-tRNA ligase activity [GO:0004812]